{
  "gene_symbol": "OR11A1",
  "gene_name": "Olfactory receptor 11A1",
  "term_label": "Unknown molecular function",
  "gene": "UniProtKB:Q9GZK7",
  "term_id": "UNKNOWN:0001"
}